{
  "gene": "UniProtKB:P51684",
  "gene_symbol": "CCR6",
  "gene_name": "C-C chemokine receptor type 6",
  "term_id": "GO:0019722",
  "term_label": "calcium-mediated signaling"
}